virus tail, shaft [GO:0098028] (cellular component) Definition: The tube of the non-contractile tails of some viruses. Sources: GOC:bm Also known as: bacteriophage tail shaft Note: This term applies in particular to the Siphoviridae bacteriophages, where the shaft is the channel for DNA translocation into the host cytoplasm. Relationships: is a type of virion component [GO:0044423]; is part of virus tail [GO:0098015]